ERBB4 signaling pathway [GO:0038130] (biological process) Definition: The series of molecular signals initiated by binding of a ligand to the tyrosine kinase receptor ERBB4 on the surface of a cell, and ending with the regulation of a downstream cellular process, e.g. transcription. Also known as: ERBB4 signalling pathway, HER4 signaling pathway, receptor tyrosine-protein kinase erbB-4 signaling pathway References: PMID:16460914 Sources: GOC:jc Regulation: negatively regulated by negative regulation of ERBB4 signaling pathway [GO:0120154] Subtypes: ERBB2-ERBB4 signaling pathway [GO:0038135], ERBB3-ERBB4 signaling pathway [GO:0038136], ERBB4-EGFR signaling pathway [GO:0038137], ERBB4-ERBB4 signaling pathway [GO:0038138] Relationships: is a type of ERBB signaling pathway [GO:0038127]